{
  "gene_symbol": "IGHG1",
  "term_label": "antigen binding",
  "gene": "UniProtKB:P01857",
  "gene_name": "Immunoglobulin heavy constant gamma 1",
  "term_id": "GO:0003823"
}